{
  "term_label": "lysosomal membrane",
  "gene": "UniProtKB:Q68CP4",
  "gene_symbol": "HGSNAT",
  "term_id": "GO:0005765",
  "gene_name": "Heparan-alpha-glucosaminide N-acetyltransferase"
}